{
  "term_label": "Unknown molecular function",
  "gene_name": "Protein FAM171A2",
  "gene_symbol": "FAM171A2",
  "term_id": "UNKNOWN:0001",
  "gene": "UniProtKB:A8MVW0"
}